{
  "gene_symbol": "GPR83",
  "term_id": "GO:0008188",
  "term_label": "neuropeptide receptor activity",
  "gene": "UniProtKB:Q9NYM4",
  "gene_name": "G-protein coupled receptor 83"
}